{
  "gene_symbol": "CSHL1",
  "gene": "UniProtKB:Q14406",
  "term_label": "animal organ development",
  "gene_name": "Chorionic somatomammotropin hormone-like 1",
  "term_id": "GO:0048513"
}